{
  "gene": "UniProtKB:Q9Y224",
  "gene_name": "RNA transcription, translation and transport factor protein",
  "term_label": "tRNA splicing, via endonucleolytic cleavage and ligation",
  "term_id": "GO:0006388",
  "gene_symbol": "RTRAF"
}